{
  "term_id": "GO:0015643",
  "term_label": "toxic substance binding",
  "gene_symbol": "TMEM181",
  "gene": "UniProtKB:Q9P2C4",
  "gene_name": "Transmembrane protein 181"
}